{
  "gene": "UniProtKB:P23560",
  "term_id": "GO:0021675",
  "gene_name": "Brain-derived neurotrophic factor",
  "gene_symbol": "BDNF",
  "term_label": "nerve development"
}